{
  "term_label": "intracellular iron ion homeostasis",
  "gene_name": "Transferrin receptor protein 1",
  "term_id": "GO:0006879",
  "gene_symbol": "TFRC",
  "gene": "UniProtKB:P02786"
}